{
  "gene_name": "Fetal and adult testis-expressed transcript protein",
  "term_label": "endoplasmic reticulum",
  "gene_symbol": "FATE1",
  "term_id": "GO:0005783",
  "gene": "UniProtKB:Q969F0"
}